{
  "term_id": "GO:0006357",
  "gene_symbol": "ETS2",
  "gene_name": "Protein C-ets-2",
  "term_label": "regulation of transcription by RNA polymerase II",
  "gene": "UniProtKB:P15036"
}